{
  "gene_symbol": "C3orf80",
  "term_label": "Unknown biological process",
  "gene_name": "Uncharacterized membrane protein C3orf80",
  "term_id": "UNKNOWN:0002",
  "gene": "UniProtKB:F5H4A9"
}